{
  "gene": "UniProtKB:Q9NZJ0",
  "gene_symbol": "DTL",
  "gene_name": "Denticleless protein homolog",
  "term_label": "nucleus",
  "term_id": "GO:0005634"
}